{
  "gene": "UniProtKB:P02655",
  "term_id": "GO:0043274",
  "gene_name": "Apolipoprotein C-II",
  "term_label": "phospholipase binding",
  "gene_symbol": "APOC2"
}